{
  "gene_symbol": "HAUS3",
  "term_label": "microtubule organizing center",
  "gene_name": "HAUS augmin-like complex subunit 3",
  "gene": "UniProtKB:Q68CZ6",
  "term_id": "GO:0005815"
}